{
  "term_id": "GO:0098703",
  "term_label": "calcium ion import across plasma membrane",
  "gene": "UniProtKB:Q13698",
  "gene_symbol": "CACNA1S",
  "gene_name": "Voltage-dependent L-type calcium channel subunit alpha-1S"
}